{
  "term_label": "3',5'-cyclic-AMP phosphodiesterase activity",
  "term_id": "GO:0004115",
  "gene": "UniProtKB:O76074",
  "gene_name": "cGMP-specific 3',5'-cyclic phosphodiesterase",
  "gene_symbol": "PDE5A"
}